regulation of secretion by asymmetric Golgi ribbon formation [GO:0090165] (biological process) Sources: GOC:ascb_2009, GOC:dph, GOC:tb Definition: The asymmetric formation of a continuous ribbon of interconnected Golgi stacks of flat cisternae that modulates the controlled release of a substance from a polarized epithelial cell. Relationships: is a type of regulation of secretion [GO:0051046]; is a type of asymmetric Golgi ribbon formation [GO:0090164]